{
  "term_id": "GO:0007029",
  "term_label": "endoplasmic reticulum organization",
  "gene_symbol": "SPTSSB",
  "gene_name": "Serine palmitoyltransferase small subunit B",
  "gene": "UniProtKB:Q8NFR3"
}